{
  "gene": "UniProtKB:Q5SQQ9",
  "term_id": "GO:0000978",
  "gene_symbol": "VAX1",
  "gene_name": "Ventral anterior homeobox 1",
  "term_label": "RNA polymerase II cis-regulatory region sequence-specific DNA binding"
}